{
  "term_label": "nucleus",
  "gene": "UniProtKB:Q96QE3",
  "gene_name": "ATPase family AAA domain-containing protein 5",
  "gene_symbol": "ATAD5",
  "term_id": "GO:0005634"
}